cell migration involved in somitogenic axis elongation [GO:0090248] (biological process) Regulation: regulated by regulation of cell migration involved in somitogenic axis elongation [GO:0090249] Also known as: cell motility involved in somitogenic axis elongation Sources: GOC:ascb_2009, GOC:dph, GOC:tb Relationships: is a type of cell migration [GO:0016477]; is part of axis elongation involved in somitogenesis [GO:0090245] Definition: Any process involved in the controlled self-propelled movement of a cell that contributes to somitogenic axis elongation.